{
  "gene_symbol": "FAM47C",
  "gene_name": "Putative protein FAM47C",
  "gene": "UniProtKB:Q5HY64",
  "term_id": "UNKNOWN:0002",
  "term_label": "Unknown biological process"
}